{
  "gene_symbol": "Q96M66",
  "term_label": "Unknown molecular function",
  "term_id": "UNKNOWN:0001",
  "gene_name": "Putative uncharacterized protein FLJ32790",
  "gene": "UniProtKB:Q96M66"
}